{
  "term_id": "GO:0006384",
  "term_label": "transcription initiation at RNA polymerase III promoter",
  "gene": "UniProtKB:Q9Y5Q8",
  "gene_name": "General transcription factor 3C polypeptide 5",
  "gene_symbol": "GTF3C5"
}